{
  "gene": "UniProtKB:Q15717",
  "term_label": "protein-RNA adaptor activity",
  "gene_symbol": "ELAVL1",
  "term_id": "GO:0140517",
  "gene_name": "ELAV-like protein 1"
}